regulation of meiotic DNA double-strand break formation [GO:1903341] (biological process) References: PMID:25103240 Sources: GOC:TermGenie, GO_REF:0000058 Subtypes: negative regulation of meiotic DNA double-strand break formation [GO:1903342], positive regulation of meiotic DNA double-strand break formation [GO:1903343], regulation of meiotic DNA double-strand break formation involved in reciprocal meiotic recombination [GO:1905261] Relationships: is a type of GO:0010564; is a type of regulation of DNA metabolic process [GO:0051052]; is a type of regulation of reproductive process [GO:2000241]; regulates meiotic DNA double-strand break formation [GO:0042138] Definition: Any process that modulates the frequency, rate or extent of meiotic DNA double-strand break formation.